{
  "gene_symbol": "EIF4EBP1",
  "gene_name": "Eukaryotic translation initiation factor 4E-binding protein 1",
  "gene": "UniProtKB:Q13541",
  "term_id": "GO:0045947",
  "term_label": "negative regulation of translational initiation"
}